prenylcysteine catabolic process [GO:0030328] (biological process) Also known as: prenylcysteine breakdown, prenylcysteine catabolism, prenylcysteine degradation Relationships: is a type of GO:0042219 Sources: GOC:ai Definition: The chemical reactions and pathways resulting in the breakdown of prenylcysteine, 3-methyl-2-buten-1-yl-cysteine, a derivative of the amino acid cysteine formed by the covalent addition of a prenyl residue.